{
  "gene": "UniProtKB:Q16772",
  "gene_symbol": "GSTA3",
  "term_id": "GO:0006805",
  "term_label": "xenobiotic metabolic process",
  "gene_name": "Glutathione S-transferase A3"
}